{
  "gene_name": "Alcohol dehydrogenase 6",
  "gene": "UniProtKB:P28332",
  "gene_symbol": "ADH6",
  "term_id": "GO:0004745",
  "term_label": "all-trans-retinol dehydrogenase (NAD+) activity"
}